{
  "gene": "UniProtKB:Q96EX3",
  "term_label": "intraciliary transport",
  "gene_symbol": "DYNC2I2",
  "gene_name": "Cytoplasmic dynein 2 intermediate chain 2",
  "term_id": "GO:0042073"
}